{
  "gene": "UniProtKB:Q7Z5A8",
  "term_label": "extracellular space",
  "gene_symbol": "TAFA3",
  "gene_name": "Chemokine-like protein TAFA-3",
  "term_id": "GO:0005615"
}